{
  "gene_name": "SR-related and CTD-associated factor 4",
  "term_label": "nucleus",
  "term_id": "GO:0005634",
  "gene_symbol": "SCAF4",
  "gene": "UniProtKB:O95104"
}